{
  "term_id": "GO:0008327",
  "term_label": "methyl-CpG binding",
  "gene": "UniProtKB:P51608",
  "gene_name": "Methyl-CpG-binding protein 2",
  "gene_symbol": "MECP2"
}